{
  "term_id": "GO:0000981",
  "gene": "UniProtKB:P52744",
  "gene_name": "Zinc finger protein 138",
  "term_label": "DNA-binding transcription factor activity, RNA polymerase II-specific",
  "gene_symbol": "ZNF138"
}